{
  "gene_symbol": "ZNF713",
  "gene_name": "Zinc finger protein 713",
  "term_id": "GO:0000978",
  "gene": "UniProtKB:Q8N859",
  "term_label": "RNA polymerase II cis-regulatory region sequence-specific DNA binding"
}